{
  "gene_name": "Cyclin-dependent kinase 16",
  "gene_symbol": "CDK16",
  "term_label": "cyclin-dependent protein serine/threonine kinase activity",
  "term_id": "GO:0004693",
  "gene": "UniProtKB:Q00536"
}